{
  "term_label": "neuropeptide signaling pathway",
  "term_id": "GO:0007218",
  "gene": "UniProtKB:P48146",
  "gene_name": "Neuropeptides B_W receptor type 2",
  "gene_symbol": "NPBWR2"
}